{
  "gene_name": "Armadillo repeat-containing protein 3",
  "gene": "UniProtKB:Q5W041",
  "term_label": "Unknown cellular component",
  "term_id": "UNKNOWN:0003",
  "gene_symbol": "ARMC3"
}